{
  "term_label": "Unknown biological process",
  "gene_name": "Arrestin domain-containing protein 2",
  "term_id": "UNKNOWN:0002",
  "gene": "UniProtKB:Q8TBH0",
  "gene_symbol": "ARRDC2"
}